{
  "gene": "UniProtKB:Q09328",
  "term_label": "alpha-1,6-mannosylglycoprotein 6-beta-N-acetylglucosaminyltransferase activity",
  "gene_symbol": "MGAT5",
  "term_id": "GO:0030144",
  "gene_name": "Alpha-1,6-mannosylglycoprotein 6-beta-N-acetylglucosaminyltransferase A"
}